{
  "term_label": "transcription repressor complex",
  "gene_name": "Insulinoma-associated protein 1",
  "gene": "UniProtKB:Q01101",
  "term_id": "GO:0017053",
  "gene_symbol": "INSM1"
}